plasma membrane pyruvate transport [GO:0006849] (biological process) Sources: GOC:ai Definition: The directed movement of pyruvate, 2-oxopropanoate, across a plasma membrane. Relationships: is a type of pyruvate transmembrane transport [GO:1901475]